{
  "term_id": "GO:0071339",
  "gene_name": "Chromodomain-helicase-DNA-binding protein 8",
  "term_label": "MLL1 complex",
  "gene_symbol": "CHD8",
  "gene": "UniProtKB:Q9HCK8"
}